{
  "term_id": "GO:0035861",
  "gene_symbol": "SMC6",
  "gene": "UniProtKB:Q96SB8",
  "gene_name": "Structural maintenance of chromosomes protein 6",
  "term_label": "site of double-strand break"
}